cellular response to hydrostatic pressure [GO:0071464] (biological process) Sources: GOC:mah Relationships: is a type of response to hydrostatic pressure [GO:0051599]; is a type of cellular response to chemical stress [GO:0062197]; is_a GO:0071462 Also known as: cellular response to biomechanical stress, cellular response to static fluid pressure Definition: Any process that results in a change in state or activity of a cell (in terms of movement, secretion, enzyme production, gene expression, etc.) as a result of a hydrostatic pressure stimulus. Hydrostatic pressure is the force acting on an object in a system where the fluid is at rest (as opposed to moving). The weight of the fluid above the object creates pressure on it.